{
  "gene_name": "Zinc finger and SCAN domain-containing protein 21",
  "term_id": "GO:0000981",
  "gene_symbol": "ZSCAN21",
  "gene": "UniProtKB:Q9Y5A6",
  "term_label": "DNA-binding transcription factor activity, RNA polymerase II-specific"
}